{
  "gene_name": "Lysosomal cobalamin transport escort protein LMBD1",
  "term_label": "protein localization to lysosome",
  "term_id": "GO:0061462",
  "gene_symbol": "LMBRD1",
  "gene": "UniProtKB:Q9NUN5"
}